{
  "gene_name": "B-cell CLL_lymphoma 6 member B protein",
  "gene": "UniProtKB:Q8N143",
  "term_label": "regulation of cell population proliferation",
  "gene_symbol": "BCL6B",
  "term_id": "GO:0042127"
}